{
  "gene": "UniProtKB:Q8WVV5",
  "term_label": "external side of plasma membrane",
  "gene_symbol": "BTN2A2",
  "term_id": "GO:0009897",
  "gene_name": "Butyrophilin subfamily 2 member A2"
}